{
  "gene_symbol": "LINC01387",
  "term_id": "UNKNOWN:0002",
  "gene": "UniProtKB:J3KSC0",
  "gene_name": "Putative uncharacterized protein encoded by LINC01387",
  "term_label": "Unknown biological process"
}